{
  "gene": "UniProtKB:Q9P2R3",
  "term_label": "endosome membrane",
  "gene_symbol": "ANKFY1",
  "term_id": "GO:0010008",
  "gene_name": "Rabankyrin-5"
}